{
  "gene_name": "High affinity choline transporter 1",
  "term_id": "GO:0030425",
  "gene": "UniProtKB:Q9GZV3",
  "gene_symbol": "SLC5A7",
  "term_label": "dendrite"
}